{
  "gene_symbol": "PPP1R14A",
  "gene_name": "Protein phosphatase 1 regulatory subunit 14A",
  "term_label": "protein serine/threonine phosphatase inhibitor activity",
  "gene": "UniProtKB:Q96A00",
  "term_id": "GO:0004865"
}